{
  "term_id": "GO:0080008",
  "gene": "UniProtKB:Q96JK2",
  "gene_symbol": "DCAF5",
  "gene_name": "DDB1- and CUL4-associated factor 5",
  "term_label": "Cul4-RING E3 ubiquitin ligase complex"
}